{
  "gene": "UniProtKB:Q9UBS0",
  "gene_name": "Ribosomal protein S6 kinase beta-2",
  "term_id": "GO:0004674",
  "gene_symbol": "RPS6KB2",
  "term_label": "protein serine/threonine kinase activity"
}